{
  "term_id": "GO:0019722",
  "gene_symbol": "CXCR2",
  "gene_name": "C-X-C chemokine receptor type 2",
  "term_label": "calcium-mediated signaling",
  "gene": "UniProtKB:P25025"
}